{
  "term_label": "positive regulation of TOR signaling",
  "gene_name": "Ragulator complex protein LAMTOR4",
  "gene": "UniProtKB:Q0VGL1",
  "term_id": "GO:0032008",
  "gene_symbol": "LAMTOR4"
}